{
  "term_label": "mitochondrial membrane",
  "gene_name": "Cytochrome c oxidase subunit 2",
  "gene_symbol": "MT-CO2",
  "gene": "UniProtKB:P00403",
  "term_id": "GO:0031966"
}